{
  "gene": "UniProtKB:B2RD01",
  "term_id": "UNKNOWN:0001",
  "gene_name": "Putative CENPB DNA-binding domain-containing protein 1",
  "gene_symbol": "CENPBD1P",
  "term_label": "Unknown molecular function"
}